{
  "gene_symbol": "AMBN",
  "gene_name": "Ameloblastin",
  "term_id": "UNKNOWN:0003",
  "term_label": "Unknown cellular component",
  "gene": "UniProtKB:Q9NP70"
}